o-dihydroxycoumarin 7-O-glucosyltransferase activity [GO:0047208] (molecular function) Definition: Catalysis of the reaction: 7,8-dihydroxycoumarin + UDP-D-glucose = daphnin + H+ + UDP. Sources: EC:2.4.1.104, RHEA:14325 Also known as: UDP-glucose:7,8-dihydroxycoumarin 7-O-beta-D-glucosyltransferase activity, UDP-glucose:o-dihydroxycoumarin glucosyltransferase activity, UDPglucose:7,8-dihydroxycoumarin 7-O-beta-D-glucosyltransferase activity, uridine diphosphoglucose-o-dihydroxycoumarin 7-O-glucosyltransferase activity Relationships: is a type of UDP-glucosyltransferase activity [GO:0035251]